{
  "gene_symbol": "VARS2",
  "gene_name": "Valine--tRNA ligase, mitochondrial",
  "gene": "UniProtKB:Q5ST30",
  "term_id": "GO:0005829",
  "term_label": "cytosol"
}